{
  "gene": "UniProtKB:A1E959",
  "gene_name": "Odontogenic ameloblast-associated protein",
  "term_label": "odontogenesis of dentin-containing tooth",
  "gene_symbol": "ODAM",
  "term_id": "GO:0042475"
}